lysosomal enzyme production involved in inflammatory response [GO:0002393] (biological process) Definition: The synthesis or release of lysosomal enzymes following a stimulus as part of a inflammatory response, resulting in an increase in intracellular or extracellular levels. Sources: GOC:add Also known as: lysosomal enzyme production involved in acute inflammatory response, production of lysosomal enzymes involved in acute inflammatory response, production of lysosomal enzymes involved in inflammatory response Relationships: is a type of GO:0002532